{
  "term_label": "Unknown biological process",
  "gene_name": "General transcription factor 3C polypeptide 4",
  "gene_symbol": "GTF3C4",
  "term_id": "UNKNOWN:0002",
  "gene": "UniProtKB:Q9UKN8"
}